{
  "term_label": "Unknown biological process",
  "term_id": "UNKNOWN:0002",
  "gene": "UniProtKB:A0A2R8YEV3",
  "gene_name": "Olfactory receptor",
  "gene_symbol": "OR2A42"
}